{
  "gene_symbol": "CCNYL2",
  "gene": "UniProtKB:Q5T2Q4",
  "term_id": "GO:0061575",
  "term_label": "cyclin-dependent protein serine/threonine kinase activator activity",
  "gene_name": "Cyclin-Y-like protein 2"
}